negative regulation of (+)-kotanin biosynthetic process [GO:1900693] (BP) Also known as: down regulation of (+)-kotanin anabolism, down regulation of (+)-kotanin biosynthesis, down regulation of (+)-kotanin biosynthetic process, down regulation of (+)-kotanin formation, down regulation of (+)-kotanin synthesis, down-regulation of (+)-kotanin anabolism, down-regulation of (+)-kotanin biosynthesis, down-regulation of (+)-kotanin biosynthetic process, down-regulation of (+)-kotanin formation, down-regulation of (+)-kotanin synthesis, downregulation of (+)-kotanin anabolism, downregulation of (+)-kotanin biosynthesis, downregulation of (+)-kotanin biosynthetic process, downregulation of (+)-kotanin formation, downregulation of (+)-kotanin synthesis, inhibition of (+)-kotanin anabolism, inhibition of (+)-kotanin biosynthesis, inhibition of (+)-kotanin formation, inhibition of (+)-kotanin synthesis, negative regulation of (+)-kotanin anabolism, negative regulation of (+)-kotanin biosynthesis, negative regulation of (+)-kotanin formation, negative regulation of (+)-kotanin synthesis, inhibition of (+)-kotanin biosynthetic process Definition: Any process that stops, prevents or reduces the frequency, rate or extent of (+)-kotanin biosynthetic process. Relationships: is a type of negative regulation of secondary metabolite biosynthetic process [GO:1900377]; is a type of regulation of (+)-kotanin biosynthetic process [GO:1900692]; negatively regulates (+)-kotanin biosynthetic process [GO:1900596] Sources: GOC:TermGenie, GOC:di